{
  "gene_symbol": "SCAMP1",
  "term_id": "GO:0006887",
  "gene": "UniProtKB:O15126",
  "term_label": "exocytosis",
  "gene_name": "Secretory carrier-associated membrane protein 1"
}